{
  "term_label": "regulation of transcription by RNA polymerase II",
  "gene": "UniProtKB:Q6P9A1",
  "gene_symbol": "ZNF530",
  "gene_name": "Zinc finger protein 530",
  "term_id": "GO:0006357"
}